{
  "term_label": "RNA polymerase II transcription regulatory region sequence-specific DNA binding",
  "term_id": "GO:0000977",
  "gene": "UniProtKB:Q6ZMY9",
  "gene_symbol": "ZNF517",
  "gene_name": "Zinc finger protein 517"
}